{
  "gene_symbol": "ITGB4",
  "gene": "UniProtKB:P16144",
  "gene_name": "Integrin beta-4",
  "term_label": "integrin binding",
  "term_id": "GO:0005178"
}